{
  "gene": "UniProtKB:Q9BW83",
  "term_id": "GO:0030992",
  "gene_name": "Intraflagellar transport protein 27 homolog",
  "term_label": "intraciliary transport particle B",
  "gene_symbol": "IFT27"
}